skeletal system morphogenesis [GO:0048705] (biological process) Definition: The process in which the anatomical structures of the skeleton are generated and organized. Also known as: skeletal morphogenesis Relationships: is a type of animal organ morphogenesis [GO:0009887]; is part of GO:0001501 Subtypes: embryonic skeletal system morphogenesis [GO:0048704] Sources: GOC:dph, GOC:dsf, GOC:jid, GOC:tb